{
  "gene_name": "F-box-like_WD repeat-containing protein TBL1Y",
  "gene": "UniProtKB:Q9BQ87",
  "term_id": "GO:0000118",
  "gene_symbol": "TBL1Y",
  "term_label": "histone deacetylase complex"
}